negative regulation of cell cycle process [GO:0010948] (biological process) Relationships: is a type of regulation of cell cycle process [GO:0010564]; is a type of negative regulation of cell cycle [GO:0045786]; negatively regulates cell cycle process [GO:0022402] Subtypes: GO:0010697, GO:0010947, negative regulation of telomere maintenance via semi-conservative replication [GO:0032214], GO:0032466, negative regulation of DNA endoreduplication [GO:0032876], negative regulation of astral microtubule depolymerization [GO:0032932], negative regulation of meiotic nuclear division [GO:0045835], negative regulation of mitotic nuclear division [GO:0045839], negative regulation of sister chromatid cohesion [GO:0045875], negative regulation of mitotic centrosome separation [GO:0046603], negative regulation of centrosome cycle [GO:0046606], GO:0051985, negative regulation of G0 to G1 transition [GO:0070317], negative regulation of ascospore formation [GO:0075297], negative regulation of cell cycle switching, mitotic to meiotic cell cycle [GO:0110045], negative regulation of chromosome attachment to the nuclear envelope [GO:0120265], negative regulation of mitotic recombination-dependent replication fork processing [GO:0120291], negative regulation of oocyte karyosome formation [GO:0120314], negative regulation of mitotic spindle assembly checkpoint signaling [GO:0140499], GO:1901988, negative regulation of nuclear cell cycle DNA replication [GO:1902576], negative regulation of mitotic spindle elongation [GO:1902845], negative regulation of centriole-centriole cohesion [GO:1903126], negative regulation of meiotic DNA double-strand break formation [GO:1903342], negative regulation of G1 to G0 transition [GO:1903451], negative regulation of centriole elongation [GO:1903723], negative regulation of meiotic cell cycle process involved in oocyte maturation [GO:1904145], negative regulation of mitotic DNA damage checkpoint [GO:1904290], negative regulation of replicative senescence [GO:1904727], negative regulation of mitotic chromosome condensation [GO:1905213], negative regulation of mitotic nuclear envelope disassembly [GO:1905558], GO:1905831 Sources: GOC:dph, GOC:tb Definition: Any process that decreases the rate, frequency or extent of a cellular process that is involved in the progression of biochemical and morphological phases and events that occur in a cell during successive cell replication or nuclear replication events.